detection of abscisic acid stimulus [GO:0009724] (biological process) Also known as: perception of abscisic acid stimulus Relationships: is a type of detection of hormone stimulus [GO:0009720]; is a type of GO:0009737 Sources: GOC:sm Definition: The series of events in which an abscisic acid stimulus is received by a cell and converted into a molecular signal.